{
  "gene_symbol": "ALG10",
  "term_label": "dolichyl pyrophosphate Glc2Man9GlcNAc2 alpha-1,2-glucosyltransferase activity",
  "gene": "UniProtKB:Q5BKT4",
  "term_id": "GO:0106073",
  "gene_name": "Dol-P-Glc:Glc(2)Man(9)GlcNAc(2)-PP-Dol alpha-1,2-glucosyltransferase"
}